{
  "term_label": "9+2 motile cilium",
  "gene_symbol": "DNAH10",
  "gene_name": "Dynein axonemal heavy chain 10",
  "term_id": "GO:0097729",
  "gene": "UniProtKB:Q8IVF4"
}